{
  "gene_name": "Annexin A4",
  "gene_symbol": "ANXA4",
  "gene": "UniProtKB:P09525",
  "term_label": "plasma membrane",
  "term_id": "GO:0005886"
}